chylomicron [GO:0042627] (cellular component) Definition: A large lipoprotein particle (diameter 75-1200 nm) composed of a central core of triglycerides and cholesterol surrounded by a protein-phospholipid coating. The proteins include one molecule of apolipoprotein B-48 and may include a variety of apolipoproteins, including APOAs, APOCs and APOE. Chylomicrons are found in blood or lymph and carry lipids from the intestines into other body tissues. References: PMID:10580165 Sources: GOC:jl, GOC:rl Subtypes: GO:0034359, GO:0034360 Relationships: is a type of GO:0034358